{
  "term_label": "RNA polymerase II cis-regulatory region sequence-specific DNA binding",
  "term_id": "GO:0000978",
  "gene": "UniProtKB:Q8N7R0",
  "gene_symbol": "NANOGP1",
  "gene_name": "Putative homeobox protein NANOG2"
}